palmitoleoyl [acyl-carrier-protein]-dependent acyltransferase activity [GO:0008951] (molecular function) Definition: Catalysis of the reaction: a palmitoleoyl-[acyl-carrier protein] + alpha-KDO-(2->4)-alpha-KDO-(2->6)-lipid IVA = KDO2-(palmitoleoyl)-lipid IVA + a holo-[acyl-carrier protein]. Sources: MetaCyc:PALMITOTRANS-RXN Relationships: is a type of acyltransferase activity, transferring groups other than amino-acyl groups [GO:0016747] Also known as: palmitoleoyl ACP-dependent acyltransferase activity